{
  "term_id": "GO:0048704",
  "gene": "UniProtKB:P17482",
  "gene_name": "Homeobox protein Hox-B9",
  "gene_symbol": "HOXB9",
  "term_label": "embryonic skeletal system morphogenesis"
}